{
  "gene_name": "DNA-directed RNA polymerase II subunit RPB4",
  "gene": "UniProtKB:O15514",
  "gene_symbol": "POLR2D",
  "term_id": "GO:0031369",
  "term_label": "translation initiation factor binding"
}